{
  "term_id": "GO:0007218",
  "term_label": "neuropeptide signaling pathway",
  "gene_symbol": "CYSLTR2",
  "gene_name": "Cysteinyl leukotriene receptor 2",
  "gene": "UniProtKB:Q9NS75"
}